ubiquitin-like protein ligase binding [GO:0044389] (molecular function) Sources: GOC:jl Definition: Binding to a ubiquitin-like protein ligase, such as ubiquitin-ligase. Also known as: E3 protein ligase binding, small conjugating protein ligase binding Subtypes: ubiquitin protein ligase binding [GO:0031625] Relationships: is a type of enzyme binding [GO:0019899]